{
  "term_label": "nucleus",
  "gene_symbol": "ZNF227",
  "gene": "UniProtKB:Q86WZ6",
  "gene_name": "Zinc finger protein 227",
  "term_id": "GO:0005634"
}